{
  "term_label": "RNA polymerase II cis-regulatory region sequence-specific DNA binding",
  "gene_name": "Zinc finger protein 486",
  "gene": "UniProtKB:Q96H40",
  "term_id": "GO:0000978",
  "gene_symbol": "ZNF486"
}